{
  "term_id": "GO:0005737",
  "gene_name": "Ubiquitin carboxyl-terminal hydrolase 3",
  "gene_symbol": "USP3",
  "gene": "UniProtKB:Q9Y6I4",
  "term_label": "cytoplasm"
}